{
  "gene_symbol": "PRRT3",
  "gene": "UniProtKB:Q5FWE3",
  "term_label": "Unknown cellular component",
  "gene_name": "Proline-rich transmembrane protein 3",
  "term_id": "UNKNOWN:0003"
}